{
  "term_id": "GO:0005737",
  "gene_name": "RING finger protein 148",
  "gene_symbol": "RNF148",
  "term_label": "cytoplasm",
  "gene": "UniProtKB:Q8N7C7"
}